{
  "gene": "UniProtKB:Q14206",
  "term_id": "GO:0008597",
  "gene_symbol": "RCAN2",
  "gene_name": "Calcipressin-2",
  "term_label": "calcium-dependent protein serine/threonine phosphatase regulator activity"
}